{
  "term_id": "GO:0002429",
  "gene": "UniProtKB:O14931",
  "term_label": "immune response-activating cell surface receptor signaling pathway",
  "gene_symbol": "NCR3",
  "gene_name": "Natural cytotoxicity triggering receptor 3"
}